{
  "gene_symbol": "RORC",
  "gene": "UniProtKB:P51449",
  "gene_name": "Nuclear receptor ROR-gamma",
  "term_id": "GO:0005634",
  "term_label": "nucleus"
}